{
  "gene": "UniProtKB:O43896",
  "gene_symbol": "KIF1C",
  "term_label": "retrograde neuronal dense core vesicle transport",
  "term_id": "GO:1990049",
  "gene_name": "Kinesin-like protein KIF1C"
}